{
  "term_label": "Unknown molecular function",
  "term_id": "UNKNOWN:0001",
  "gene_symbol": "WDPCP",
  "gene": "UniProtKB:O95876",
  "gene_name": "WD repeat-containing and planar cell polarity effector protein fritz homolog"
}